{
  "gene": "UniProtKB:Q8N9R0",
  "term_label": "Unknown cellular component",
  "gene_symbol": "LINC00304",
  "gene_name": "Putative uncharacterized protein encoded by LINC00304",
  "term_id": "UNKNOWN:0003"
}